{
  "gene_name": "Plasmanylethanolamine desaturase 1",
  "term_id": "GO:0050207",
  "gene_symbol": "PEDS1",
  "term_label": "plasmanylethanolamine desaturase activity",
  "gene": "UniProtKB:A5PLL7"
}